{
  "gene_name": "Transmembrane protein 26",
  "term_label": "Unknown cellular component",
  "term_id": "UNKNOWN:0003",
  "gene_symbol": "TMEM26",
  "gene": "UniProtKB:Q6ZUK4"
}